{
  "term_id": "GO:0031122",
  "term_label": "cytoplasmic microtubule organization",
  "gene": "UniProtKB:Q9P219",
  "gene_name": "Protein Daple",
  "gene_symbol": "CCDC88C"
}